negative regulation of plasmacytoid dendritic cell cytokine production [GO:0002737] (biological process) Also known as: down regulation of plasmacytoid dendritic cell cytokine production, down-regulation of plasmacytoid dendritic cell cytokine production, downregulation of plasmacytoid dendritic cell cytokine production, inhibition of plasmacytoid dendritic cell cytokine production Definition: Any process that stops, prevents, or reduces the frequency, rate, or extent of plasmacytoid dendritic cell cytokine production. Relationships: is a type of GO:0002731; is a type of regulation of plasmacytoid dendritic cell cytokine production [GO:0002736]; negatively regulates GO:0002373 Sources: GOC:add